{
  "term_id": "GO:0051015",
  "gene_symbol": "MYO19",
  "gene": "UniProtKB:Q96H55",
  "term_label": "actin filament binding",
  "gene_name": "Unconventional myosin-XIX"
}